{
  "gene_name": "Putative postmeiotic segregation increased 2-like protein 11",
  "gene": "UniProtKB:Q13670",
  "term_id": "UNKNOWN:0003",
  "term_label": "Unknown cellular component",
  "gene_symbol": "PMS2P11"
}